{
  "gene_symbol": "OR2B2",
  "gene_name": "Olfactory receptor 2B2",
  "term_id": "GO:0005886",
  "term_label": "plasma membrane",
  "gene": "UniProtKB:Q9GZK3"
}